{
  "term_id": "GO:0099560",
  "gene": "UniProtKB:Q9HCJ2",
  "gene_symbol": "LRRC4C",
  "term_label": "synaptic membrane adhesion",
  "gene_name": "Leucine-rich repeat-containing protein 4C"
}